{
  "term_label": "E-box binding",
  "gene_name": "Class E basic helix-loop-helix protein 23",
  "gene": "UniProtKB:Q8NDY6",
  "gene_symbol": "BHLHE23",
  "term_id": "GO:0070888"
}